{
  "term_id": "GO:0030020",
  "gene_symbol": "COL16A1",
  "gene": "UniProtKB:Q07092",
  "gene_name": "Collagen alpha-1(XVI) chain",
  "term_label": "extracellular matrix structural constituent conferring tensile strength"
}